{
  "term_id": "GO:0097193",
  "gene_symbol": "CARD8",
  "term_label": "intrinsic apoptotic signaling pathway",
  "gene": "UniProtKB:Q9Y2G2",
  "gene_name": "Caspase recruitment domain-containing protein 8"
}